{
  "term_label": "homophilic cell-cell adhesion",
  "term_id": "GO:0007156",
  "gene_name": "Myopalladin",
  "gene": "UniProtKB:Q86TC9",
  "gene_symbol": "MYPN"
}